{
  "gene_name": "Forkhead box protein D4-like 3",
  "term_label": "RNA polymerase II cis-regulatory region sequence-specific DNA binding",
  "gene_symbol": "FOXD4L3",
  "gene": "UniProtKB:Q6VB84",
  "term_id": "GO:0000978"
}